sedoheptulose-bisphosphatase activity [GO:0050278] (molecular function) Sources: EC:3.1.3.37, MetaCyc:SEDOHEPTULOSE-BISPHOSPHATASE-RXN Also known as: SBPase activity, sedoheptulose 1,7-bisphosphatase activity, sedoheptulose 1,7-diphosphatase activity, sedoheptulose 1,7-diphosphate phosphatase activity, sedoheptulose bisphosphatase activity, sedoheptulose diphosphatase activity, sedoheptulose-1,7-bisphosphatase activity, sedoheptulose-1,7-bisphosphate 1-phosphohydrolase activity Relationships: is a type of phosphatase activity [GO:0016791] Definition: Catalysis of the reaction: sedoheptulose 1,7-bisphosphate + H2O = sedoheptulose 7-phosphate + phosphate.